basal layer of collagen and cuticulin-based cuticle extracellular matrix [GO:0060110] (cellular component) Definition: The layer of cuticle most closely apposed to the hypodermal cells. The morphology of the basal layer varies with life stage. In adult C. elegans animals, the basal layers is comprised of three sublayers: two fibrous layers whose fibers run in clockwise and counter-clockwise directions meeting one another at a 60 degree angle, and an amorphous basal layer that lies underneath the fibrous layers and directly contacts the hypodermis. In C. elegans dauer and L1 larval stage animals, the basal layer is characterized by a striated pattern that appears to derive from interwoven laminae. An example of this component is found in Caenorhabditis elegans. Relationships: is_a cellular anatomical structure [GO:0110165]; is part of GO:0060102 Also known as: basal layer of collagen and cuticulin-based exoskeleton extracellular matrix Sources: GOC:dph, GOC:kmv, ISSN:15518507